regulation of metanephric nephron tubule epithelial cell differentiation [GO:0072307] (biological process) Relationships: is a type of GO:0072182; regulates metanephric nephron tubule epithelial cell differentiation [GO:0072257] Sources: GOC:mtg_kidney_jan10 Definition: Any process that modulates the frequency, rate or extent of metanephric nephron tubule epithelial cell differentiation. Subtypes: negative regulation of metanephric nephron tubule epithelial cell differentiation [GO:0072308]